{
  "gene_name": "Putative uncharacterized protein ASB16-AS1",
  "term_label": "Unknown molecular function",
  "term_id": "UNKNOWN:0001",
  "gene": "UniProtKB:Q495Z4",
  "gene_symbol": "ASB16-AS1"
}